{
  "term_label": "Unknown molecular function",
  "term_id": "UNKNOWN:0001",
  "gene": "UniProtKB:Q6ZUX7",
  "gene_symbol": "LHFPL2",
  "gene_name": "LHFPL tetraspan subfamily member 2 protein"
}